{
  "gene": "UniProtKB:Q96Q11",
  "gene_symbol": "TRNT1",
  "gene_name": "CCA tRNA nucleotidyltransferase 1, mitochondrial",
  "term_label": "mitochondrion",
  "term_id": "GO:0005739"
}